cellular response to platelet-derived growth factor stimulus [GO:0036120] (biological process) Sources: GOC:yaf Definition: Any process that results in a change in state or activity of a cell (in terms of movement, secretion, enzyme production, gene expression, etc.) as a result of a platelet-derived growth factor stimulus. Relationships: is a type of response to platelet-derived growth factor [GO:0036119]; is a type of cellular response to growth factor stimulus [GO:0071363] Also known as: cellular response to PDGF stimulus